{
  "gene_symbol": "MROH7",
  "gene": "UniProtKB:Q68CQ1",
  "term_label": "Unknown molecular function",
  "term_id": "UNKNOWN:0001",
  "gene_name": "Maestro heat-like repeat-containing protein family member 7"
}